{
  "term_id": "GO:0000785",
  "gene": "UniProtKB:Q16650",
  "gene_symbol": "TBR1",
  "term_label": "chromatin",
  "gene_name": "T-box brain protein 1"
}